exocyst localization [GO:0051601] (biological process) Subtypes: regulation of endocytosis by exocyst localization [GO:0051600] Definition: Any process in which an exocyst is transported to, or maintained in, a specific location. An exocyst is a protein complex peripherally associated with the plasma membrane that determines where vesicles dock and fuse. Sources: GOC:ai Relationships: is_a protein-containing complex localization [GO:0031503] Also known as: establishment and maintenance of exocyst localization, exocyst localisation Regulation: regulated by regulation of exocyst localization [GO:0060178]